{
  "gene_symbol": "ZIC2",
  "term_label": "nucleus",
  "gene": "UniProtKB:O95409",
  "term_id": "GO:0005634",
  "gene_name": "Zinc finger protein ZIC 2"
}